{
  "term_label": "regulation of transcription by RNA polymerase II",
  "term_id": "GO:0006357",
  "gene_symbol": "PRDM11",
  "gene": "UniProtKB:Q9NQV5",
  "gene_name": "PR domain-containing protein 11"
}